{
  "gene_symbol": "ARHGEF18",
  "gene": "UniProtKB:Q6ZSZ5",
  "gene_name": "Rho guanine nucleotide exchange factor 18",
  "term_id": "GO:0005085",
  "term_label": "guanyl-nucleotide exchange factor activity"
}